extrinsic apoptotic signaling pathway via death domain receptors [GO:0008625] (biological process) Definition: The series of molecular signals in which a signal is conveyed from the cell surface to trigger the apoptotic death of a cell. The pathway starts with a ligand binding to a death domain receptor on the cell surface, and ends when the execution phase of apoptosis is triggered. Sources: GOC:mah, GOC:mtg_apoptosis Relationships: is a type of extrinsic apoptotic signaling pathway [GO:0097191] Regulation: regulated by regulation of extrinsic apoptotic signaling pathway via death domain receptors [GO:1902041]; RO_0002212 by negative regulation of extrinsic apoptotic signaling pathway via death domain receptors [GO:1902042]; positively regulated by GO:1902043 Subtypes: TRAIL-activated apoptotic signaling pathway [GO:0036462] Also known as: induction of apoptosis via death receptors, death receptor-mediated apoptosis, induction of apoptosis via death domain receptors Note: Gene products that may be annotated to this term include: 1) ligands such as FASL; 2) receptors such as FAS/CD95 (though care should be taken because FAS can also act as a non-apoptotic signal transducer); 3) signaling molecules such as FADD (FAS-associated protein with a death domain), cIAPs (cellular inhibitor of apoptosis proteins), c-FLIPs and caspases 8 and 10. Examples are TWEAK (TNF12) and FN14 (TNFRSF12A) (UniProt symbols O43508 and Q9NP84) in PMID:21525013.